post-translational protein targeting to membrane, translocation [GO:0031204] (biological process) Regulation: regulated by regulation of post-translational protein targeting to membrane, translocation [GO:0120235]; negatively regulated by negative regulation of post-translational protein targeting to membrane, translocation [GO:0120236] Relationships: is a type of intracellular protein transmembrane transport [GO:0065002]; is part of post-translational protein targeting to endoplasmic reticulum membrane [GO:0006620] Definition: The process in which a protein translocates through the ER membrane posttranslationally. Also known as: posttranslational protein membrane targeting, translocation, posttranslational protein targeting to membrane, translocation, protein translocation during posttranslational protein targeting to membrane References: PMID:12518317, PMID:8707814